regulation of protein K48-linked ubiquitination [GO:0061945] (biological process) References: PMID:23460740 Definition: Any process that modulates the rate, frequency or extent of protein K-48-linked ubiquitination, a protein ubiquitination process in which a polymer of ubiquitin, formed by linkages between lysine residues at position 48 of the ubiquitin monomers, is added to a protein. K48-linked ubiquitination targets the substrate protein for degradation. Subtypes: negative regulation of protein K48-linked ubiquitination [GO:0061944], positive regulation of protein K48-linked ubiquitination [GO:1902524] Relationships: is a type of regulation of protein polyubiquitination [GO:1902914]; regulates protein K48-linked ubiquitination [GO:0070936]